{
  "term_label": "Golgi apparatus",
  "gene_symbol": "PLOD3",
  "term_id": "GO:0005794",
  "gene": "UniProtKB:O60568",
  "gene_name": "Multifunctional procollagen lysine hydroxylase and glycosyltransferase LH3"
}